{
  "gene_name": "Probable ubiquitin carboxyl-terminal hydrolase FAF-Y",
  "gene_symbol": "USP9Y",
  "term_label": "cytosol",
  "term_id": "GO:0005829",
  "gene": "UniProtKB:O00507"
}